N(alpha)-benzyloxycarbonylleucine hydrolase activity [GO:0047413] (molecular function) Definition: Catalysis of the reaction: N-benzyloxycarbonyl-L-leucine + H2O + H+ = L-leucine + benzyl alcohol + CO2. Sources: EC:3.5.1.64, RHEA:18901 Also known as: alpha-N-benzyloxycarbonyl-L-leucine urethanehydrolase activity, benzyloxycarbonylleucine hydrolase activity, nalpha-benzyloxycarbonyl amino acid urethane hydrolase IV, nalpha-benzyloxycarbonyl-L-leucine urethanehydrolase activity, nalpha-benzyloxycarbonylleucine hydrolase activity Relationships: is a type of hydrolase activity, acting on carbon-nitrogen (but not peptide) bonds, in linear amides [GO:0016811]